{
  "gene_name": "Immunoglobulin superfamily member 21",
  "term_id": "GO:0099550",
  "gene_symbol": "IGSF21",
  "gene": "UniProtKB:Q96ID5",
  "term_label": "trans-synaptic signaling, modulating synaptic transmission"
}